{
  "gene_name": "Tetratricopeptide repeat protein 21B",
  "term_id": "GO:0030991",
  "gene_symbol": "TTC21B",
  "term_label": "intraciliary transport particle A",
  "gene": "UniProtKB:Q7Z4L5"
}